{
  "gene_symbol": "LURAP1",
  "gene_name": "Leucine rich adaptor protein 1",
  "term_label": "positive regulation of canonical NF-kappaB signal transduction",
  "gene": "UniProtKB:Q96LR2",
  "term_id": "GO:0043123"
}